{
  "gene_name": "Teashirt homolog 2",
  "term_id": "GO:0000981",
  "gene": "UniProtKB:Q9NRE2",
  "term_label": "DNA-binding transcription factor activity, RNA polymerase II-specific",
  "gene_symbol": "TSHZ2"
}